{
  "gene_symbol": "ULBP3",
  "gene": "UniProtKB:Q9BZM4",
  "gene_name": "UL16-binding protein 3",
  "term_label": "extracellular space",
  "term_id": "GO:0005615"
}